{
  "gene": "UniProtKB:Q9BVV7",
  "gene_name": "Mitochondrial import inner membrane translocase subunit Tim21",
  "term_label": "TIM23 mitochondrial import inner membrane translocase complex",
  "term_id": "GO:0005744",
  "gene_symbol": "TIMM21"
}